SUMO-modified protein reader activity [GO:0140037] (molecular function) Definition: A molecular adaptor that recognizes and binds a target protein containing a SUMO modification and that brings the target protein into contact with another protein to allow those proteins to function in a coordinated way. References: PMID:26060076 Also known as: SUMO-dependent protein binding Note: This term should only be used when the binding is shown to require sumoylation of the target protein: the interaction needs to be tested with and without the PTM. The binding does not need to be at the site of sumoylation. It may be that the sumoylation causes a conformational change that allows binding of the protein to another region; this type of sumoylation-dependent protein binding is valid for annotation to this term. Relationships: is a type of ubiquitin-like protein reader activity [GO:0140035]